{
  "gene_name": "Alpha-2-macroglobulin receptor-associated protein",
  "term_label": "negative regulation of receptor internalization",
  "term_id": "GO:0002091",
  "gene_symbol": "LRPAP1",
  "gene": "UniProtKB:P30533"
}